{
  "gene_symbol": "OR52W1",
  "gene_name": "Olfactory receptor 52W1",
  "term_label": "Unknown biological process",
  "term_id": "UNKNOWN:0002",
  "gene": "UniProtKB:Q6IF63"
}